{
  "gene_symbol": "MMP16",
  "term_id": "GO:0005615",
  "term_label": "extracellular space",
  "gene_name": "Matrix metalloproteinase-16",
  "gene": "UniProtKB:P51512"
}